{
  "gene_name": "Palmitoyltransferase ZDHHC15",
  "term_label": "protein-cysteine S-palmitoyltransferase activity",
  "gene_symbol": "ZDHHC15",
  "gene": "UniProtKB:Q96MV8",
  "term_id": "GO:0019706"
}